beta-glucoside transmembrane transporter activity [GO:0015573] (molecular function) Relationships: is a type of glucoside transmembrane transporter activity [GO:0042947]; is part of beta-glucoside transport [GO:0015759] Also known as: beta-glucoside permease activity Definition: Enables the transfer of beta-glucosides from one side of a membrane to the other. Beta-glucosides are glycosides in which the sugar group is a glucose residue, and the anomeric carbon of the bond is in a beta configuration. Subtypes: protein-N(PI)-phosphohistidine-beta-glucoside phosphotransferase system transporter activity [GO:0022882], salicin transmembrane transporter activity [GO:0042950], arbutin transmembrane transporter activity [GO:0042951] References: PMID:7883710 Sources: GOC:jl, GOC:mtg_transport, ISBN:0198506732, ISBN:0815340729